regulation of cell maturation [GO:1903429] (biological process) Relationships: is_a regulation of cell development [GO:0060284]; RO_0002211 GO:0048469 Also known as: regulation of functional differentiation References: PMID:17459944 Sources: GOC:TermGenie, GO_REF:0000058 Subtypes: regulation of neuron maturation [GO:0014041], regulation of erythrocyte enucleation [GO:0061930], regulation of oocyte maturation [GO:1900193], regulation of sperm capacitation [GO:1902490], negative regulation of cell maturation [GO:1903430], positive regulation of cell maturation [GO:1903431] Definition: Any process that modulates the frequency, rate or extent of cell maturation.